{
  "term_id": "GO:0008478",
  "gene": "UniProtKB:O00764",
  "gene_symbol": "PDXK",
  "gene_name": "Pyridoxal kinase",
  "term_label": "pyridoxal kinase activity"
}